{
  "term_label": "proteolysis",
  "gene_symbol": "ADAM23",
  "gene_name": "Disintegrin and metalloproteinase domain-containing protein 23",
  "term_id": "GO:0006508",
  "gene": "UniProtKB:O75077"
}